cellular response to cycloheximide [GO:0071409] (BP) Sources: GOC:mah Relationships: is a type of response to cycloheximide [GO:0046898]; is a type of cellular response to alcohol [GO:0097306]; is_a cellular response to ketone [GO:1901655]; is a type of GO:1901699 Definition: Any process that results in a change in state or activity of a cell (in terms of movement, secretion, enzyme production, gene expression, etc.) as a result of a cycloheximide stimulus. Cycloheximide (actidione) is an antibiotic produced by some Streptomyces species which interferes with protein synthesis in eukaryotes. Also known as: cellular response to actidione